isoprenoid biosynthetic process via mevalonate [GO:1902767] (biological process) Relationships: is a type of isoprenoid biosynthetic process [GO:0008299] Subtypes: GO:0010142 References: PMID:11078528 Sources: GOC:TermGenie, GOC:mengo_curators, GO_REF:0000092 Definition: The chemical reactions and pathways resulting in the formation of isoprenoid via mevalonate. Also known as: isoprenoid anabolism via mevalonate, isoprenoid biosynthesis via mevalonate, isoprenoid formation via mevalonate, isoprenoid synthesis via mevalonate